symbiont-mediated suppression of host innate immune response [GO:0052170] (biological process) Also known as: negative regulation of innate immune response in other organism, down regulation by symbiont of host innate immunity, down-regulation by symbiont of host innate immunity, downregulation by symbiont of host innate immunity, negative regulation by symbiont of host innate immune response, negative regulation by symbiont of host innate immunity, negative regulation of host innate immune response, suppression by symbiont of host innate immune response, suppression of host innate immune response, inhibition by symbiont of host innate immunity Relationships: is a type of symbiont-mediated perturbation of host innate immune response [GO:0052167]; is a type of symbiont-mediated suppression of host immune response [GO:0052562] Sources: GOC:mtg_pamgo_17jul06 Definition: A process in which a symbiont inhibits or disrupts the normal execution of the innate immune response of the host organism, the host's first line of defense against infection. The host is defined as the larger of the organisms involved in a symbiotic interaction. Subtypes: GO:0039560, symbiont-mediated suppression of host JAK-STAT cascade via inhibition of host TYK2 activity [GO:0039574], symbiont-mediated suppression of host ISG15-protein conjugation [GO:0039579], symbiont-mediated suppression of host complement activation [GO:0042784], symbiont-mediated suppression of host pathogen-associated molecular pattern receptor signaling pathway [GO:0052078], effector-mediated suppression of host innate immune response [GO:0140403], GO:0140533